{
  "term_id": "UNKNOWN:0003",
  "gene": "UniProtKB:A0A075B7E0",
  "term_label": "Unknown cellular component",
  "gene_symbol": "IGHD3OR15-3B",
  "gene_name": "Protein IGHD3OR15-3A (Fragment)"
}